{
  "gene_name": "Adropin",
  "gene_symbol": "ENHO",
  "gene": "UniProtKB:Q6UWT2",
  "term_label": "plasma membrane",
  "term_id": "GO:0005886"
}